{
  "gene_symbol": "CRIPTO3",
  "gene_name": "Putative teratocarcinoma-derived growth factor 3",
  "term_label": "activin receptor binding",
  "gene": "UniProtKB:P51864",
  "term_id": "GO:0070697"
}